{
  "gene": "UniProtKB:Q9BUV8",
  "term_id": "UNKNOWN:0003",
  "gene_name": "GEL complex subunit OPTI",
  "gene_symbol": "RAB5IF",
  "term_label": "Unknown cellular component"
}